{
  "gene_name": "Protein SIX6OS1",
  "term_label": "oogenesis",
  "gene": "UniProtKB:Q8N1H7",
  "gene_symbol": "SIX6OS1",
  "term_id": "GO:0048477"
}